perinuclear theca [GO:0033011] (cellular component) Definition: A condensed cytoplasmic structure that covers the nucleus of mammalian spermatozoa except for a narrow zone around the insertion of the tail. It shows two distinct regions, a subacrosomal layer and, continuing caudally beyond the acrosomic system, the postacrosomal sheath. The perinuclear theca has been considered a cytoskeletal scaffold responsible for maintaining the overall architecture of the mature sperm head; however, recent studies indicate that the bulk of its constituent proteins are not traditional cytoskeletal proteins but rather a variety of cytosolic proteins. Relationships: is a type of cytoskeleton [GO:0005856]; is part of perinuclear region of cytoplasm [GO:0048471] References: PMID:17289678, PMID:8025156